regulation of chemokine (C-C motif) ligand 4 production [GO:0071643] (biological process) Definition: Any process that modulates the frequency, rate, or extent of production of chemokine (C-C motif) ligand 4. Subtypes: negative regulation of chemokine (C-C motif) ligand 4 production [GO:0071644], positive regulation of chemokine (C-C motif) ligand 4 production [GO:0071645] Relationships: is a type of regulation of chemokine production [GO:0032642]; regulates chemokine (C-C motif) ligand 4 production [GO:0071606] Sources: GOC:mah Also known as: regulation of macrophage inflammatory protein production, regulation of CCL4 production, regulation of MIP-1b production